{
  "gene": "UniProtKB:Q9NX00",
  "term_id": "UNKNOWN:0003",
  "gene_name": "Transmembrane protein 160",
  "term_label": "Unknown cellular component",
  "gene_symbol": "TMEM160"
}